{
  "gene_symbol": "FGF18",
  "term_id": "GO:0030334",
  "gene": "UniProtKB:O76093",
  "gene_name": "Fibroblast growth factor 18",
  "term_label": "regulation of cell migration"
}